{
  "gene_symbol": "KCNQ1",
  "gene": "UniProtKB:P51787",
  "term_label": "membrane",
  "gene_name": "Potassium voltage-gated channel subfamily KQT member 1",
  "term_id": "GO:0016020"
}